{
  "gene_symbol": "CD109",
  "term_label": "Unknown molecular function",
  "term_id": "UNKNOWN:0001",
  "gene": "UniProtKB:Q6YHK3",
  "gene_name": "CD109 antigen"
}